isoursodeoxycholate 7-beta-dehydrogenase (NAD+) activity [GO:0106282] (molecular function) Relationships: is_a GO:0033764 Definition: Catalysis of the reaction: 3-beta,7-beta-dihydroxy-5-beta-cholan-24-oate + NAD+ = 3-beta-hydroxy-7-oxo-5-beta-cholan-24-oate + H+ + NADH. References: PMID:12917011 Sources: RHEA:42024